{
  "gene": "UniProtKB:P56373",
  "term_id": "GO:0005886",
  "gene_symbol": "P2RX3",
  "gene_name": "P2X purinoceptor 3",
  "term_label": "plasma membrane"
}